myosin XVII complex [GO:0031487] (cellular component) Relationships: is a type of unconventional myosin complex [GO:0016461] References: PMID:24443438 Definition: A myosin complex containing one or more class XVII myosin heavy chains and associated light chains.